{
  "gene": "UniProtKB:Q8IYR2",
  "gene_symbol": "SMYD4",
  "term_id": "GO:0007507",
  "gene_name": "SET and MYND domain-containing protein 4",
  "term_label": "heart development"
}